{
  "gene": "UniProtKB:Q8IUA0",
  "term_label": "Unknown cellular component",
  "term_id": "UNKNOWN:0003",
  "gene_symbol": "WFDC8",
  "gene_name": "WAP four-disulfide core domain protein 8"
}